{
  "gene_symbol": "KRTAP5-5",
  "gene": "UniProtKB:Q701N2",
  "gene_name": "Keratin-associated protein 5-5",
  "term_label": "Unknown biological process",
  "term_id": "UNKNOWN:0002"
}